regulation of transmission of nerve impulse [GO:0051969] (biological process) Relationships: is a type of regulation of cell communication [GO:0010646]; is a type of regulation of nervous system process [GO:0031644]; regulates transmission of nerve impulse [GO:0019226] Subtypes: GO:0051970, positive regulation of transmission of nerve impulse [GO:0051971], regulation of neuronal action potential [GO:0098908] Sources: GOC:ai Also known as: regulation of conduction of nerve impulse Definition: Any process that modulates the frequency, rate or extent of transmission of a nerve impulse, the sequential electrochemical polarization and depolarization that travels across the membrane of a neuron in response to stimulation.